{
  "gene_symbol": "CD34",
  "term_label": "Unknown cellular component",
  "gene": "UniProtKB:P28906",
  "term_id": "UNKNOWN:0003",
  "gene_name": "Hematopoietic progenitor cell antigen CD34"
}